{
  "term_id": "UNKNOWN:0002",
  "gene_name": "Transcription factor IIIB 50 kDa subunit",
  "gene_symbol": "BRF2",
  "gene": "UniProtKB:Q9HAW0",
  "term_label": "Unknown biological process"
}